{
  "gene_symbol": "SIRPG",
  "term_id": "GO:0050870",
  "gene_name": "Signal-regulatory protein gamma",
  "term_label": "positive regulation of T cell activation",
  "gene": "UniProtKB:Q9P1W8"
}